{
  "term_id": "UNKNOWN:0001",
  "term_label": "Unknown molecular function",
  "gene_name": "Cell adhesion molecule 3",
  "gene_symbol": "CADM3",
  "gene": "UniProtKB:Q8N126"
}